{
  "gene_name": "Forkhead box protein I2",
  "gene_symbol": "FOXI2",
  "term_id": "GO:0030154",
  "gene": "UniProtKB:Q6ZQN5",
  "term_label": "cell differentiation"
}